regulation of grooming behavior [GO:2000821] (BP) Relationships: is a type of regulation of behavior [GO:0050795]; RO_0002211 grooming behavior [GO:0007625] Sources: GOC:BHF Definition: Any process that modulates the frequency, rate or extent of grooming behavior. Also known as: regulation of grooming behaviour